{
  "term_id": "GO:0052751",
  "gene_symbol": "NUDT22",
  "gene": "UniProtKB:Q9BRQ3",
  "term_label": "GDP-mannose hydrolase activity",
  "gene_name": "Uridine diphosphate glucose pyrophosphatase NUDT22"
}